{
  "term_label": "aspartate biosynthetic process",
  "gene_name": "Putative aspartate aminotransferase, cytoplasmic 2",
  "gene": "UniProtKB:Q8NHS2",
  "term_id": "GO:0006532",
  "gene_symbol": "GOT1L1"
}